{
  "gene": "UniProtKB:Q9NX01",
  "term_label": "U5 snRNP",
  "term_id": "GO:0005682",
  "gene_name": "Thioredoxin-like protein 4B",
  "gene_symbol": "TXNL4B"
}